symbiont-mediated suppression of host cytoplasmic pattern recognition receptor signaling pathway via inhibition of IRF7 activity [GO:0039557] (biological process) Note: This term is for annotation of symbiont proteins that counteract the host anti-microbial innate immune response. Also known as: suppression by virus of host viral-induced cytoplasmic pattern recognition receptor signaling pathway via inhibition of IRF7 activity, inhibition of host IRF7 by virus, inhibition of host interferon regulatory factor-7 by virus, suppression by virus of host IRF7 activity, suppression by virus of host interferon regulatory factor 7 activity References: PMID:11943871, PMID:16014964, PMID:19557165 Relationships: is a type of symbiont-mediated suppression of cytoplasmic pattern recognition receptor signaling pathway [GO:0039537] Definition: A process in which a symbiont interferes with, inhibits or disrupts a cytoplasmic pattern recognition receptor signaling pathway by reducing the activity of IRF7 (interferon regulatory factor-7). IRF7 a transcription factor in the RIG-I/MDA-5 signaling pathway. Viral infection triggers phosphorylation of cytoplasmic IRF7, which allows IRF7 to form a homodimer, migrate to the nucleus, and activate transcription of IFN-alpha and IFN-beta genes.